{
  "gene": "UniProtKB:O75197",
  "gene_name": "Low-density lipoprotein receptor-related protein 5",
  "term_id": "UNKNOWN:0001",
  "gene_symbol": "LRP5",
  "term_label": "Unknown molecular function"
}